{
  "gene": "UniProtKB:Q8IZ41",
  "term_id": "GO:0005829",
  "gene_name": "Ras and EF-hand domain-containing protein",
  "gene_symbol": "RASEF",
  "term_label": "cytosol"
}